{
  "term_id": "GO:0005085",
  "gene_symbol": "PCP2",
  "gene_name": "Purkinje cell protein 2 homolog",
  "gene": "UniProtKB:Q8IVA1",
  "term_label": "guanyl-nucleotide exchange factor activity"
}